{
  "term_id": "GO:0008479",
  "gene_name": "Queuine tRNA-ribosyltransferase catalytic subunit 1",
  "gene": "UniProtKB:Q9BXR0",
  "gene_symbol": "QTRT1",
  "term_label": "tRNA-guanosine(34) queuine transglycosylase activity"
}